protein localization to cell division site after cytokinesis [GO:0098841] (biological process) References: PMID:25411334 Definition: A cellular protein localization process in which a protein is transported to, or maintained at, the site of cell division following cytokinesis. Relationships: is a type of GO:0072741